{
  "gene": "UniProtKB:Q9UGM5",
  "gene_symbol": "FETUB",
  "term_id": "GO:0007339",
  "term_label": "binding of sperm to zona pellucida",
  "gene_name": "Fetuin-B"
}